aminophospholipid flippase activity [GO:0015247] (molecular function) Definition: Enables the transfer of aminophospholipids from the exoplasmic to the cytosolic leaflet of a membrane, using energy from the hydrolysis of ATP. Aminophospholipids contain phosphoric acid as a mono- or diester and an amino (NH2) group. Subtypes: GO:0140346 Also known as: aminophospholipid transmembrane transporter activity, aminophospholipid transporter activity Relationships: is a type of phospholipid transporter activity [GO:0005548]; is a type of flippase activity [GO:0140327]; BFO_0000050 aminophospholipid translocation [GO:0140331] Sources: GOC:pg